{
  "gene": "UniProtKB:Q6ZNR0",
  "gene_symbol": "TMEM91",
  "gene_name": "Transmembrane protein 91",
  "term_label": "Unknown molecular function",
  "term_id": "UNKNOWN:0001"
}